{
  "gene_symbol": "HIRA",
  "term_label": "nucleosome binding",
  "gene": "UniProtKB:P54198",
  "term_id": "GO:0031491",
  "gene_name": "Protein HIRA"
}